{
  "term_label": "cytokine binding",
  "term_id": "GO:0019955",
  "gene": "UniProtKB:P26951",
  "gene_name": "Interleukin-3 receptor subunit alpha",
  "gene_symbol": "IL3RA"
}